steroid hormone biosynthetic process [GO:0120178] (biological process) Definition: The chemical reactions and pathways resulting in the formation of any steroid hormone, naturally occurring substances secreted by specialized cells that affects the metabolism or behavior of other cells possessing functional receptors for the hormone. Subtypes: C21-steroid hormone biosynthetic process [GO:0006700], androgen biosynthetic process [GO:0006702], GO:0006703, GO:0006704, mineralocorticoid biosynthetic process [GO:0006705], vitamin D3 biosynthetic process [GO:1901755] Relationships: is a type of steroid biosynthetic process [GO:0006694] Sources: GOC:krc, GOC:nln